{
  "term_label": "Unknown molecular function",
  "gene_name": "Keratin-associated protein 26-1",
  "gene": "UniProtKB:Q6PEX3",
  "term_id": "UNKNOWN:0001",
  "gene_symbol": "KRTAP26-1"
}